{
  "term_label": "barbed-end actin filament capping",
  "term_id": "GO:0051016",
  "gene_name": "Macrophage-capping protein",
  "gene_symbol": "CAPG",
  "gene": "UniProtKB:P40121"
}